[hydroxymethylglutaryl-CoA reductase (NADPH)]-phosphatase activity [GO:0047384] (molecular function) Also known as: reductase phosphatase activity, hydroxymethylglutaryl-CoA reductase (NADPH)-phosphatase activity, hydroxymethylglutaryl-CoA reductase (NADPH)-phosphate phosphohydrolase activity Definition: Catalysis of the reaction: H2O + [hydroxymethylglutaryl-CoA reductase (NADPH)] phosphate = phosphate + [hydroxymethylglutaryl-CoA reductase (NADPH)]. Relationships: is a type of phosphoprotein phosphatase activity [GO:0004721] Sources: EC:3.1.3.47, MetaCyc:3.1.3.47-RXN